{
  "gene_symbol": "AP5B1",
  "gene": "UniProtKB:Q2VPB7",
  "term_label": "Unknown molecular function",
  "term_id": "UNKNOWN:0001",
  "gene_name": "AP-5 complex subunit beta-1"
}